{
  "gene_symbol": "CRIM1",
  "term_label": "Unknown cellular component",
  "term_id": "UNKNOWN:0003",
  "gene_name": "Cysteine-rich motor neuron 1 protein",
  "gene": "UniProtKB:Q9NZV1"
}